{
  "gene": "UniProtKB:P43681",
  "gene_name": "Neuronal acetylcholine receptor subunit alpha-4",
  "term_label": "presynaptic modulation of chemical synaptic transmission",
  "gene_symbol": "CHRNA4",
  "term_id": "GO:0099171"
}